regulation of sporulation resulting in formation of a cellular spore [GO:0042173] (biological process) Sources: GOC:jl Subtypes: negative regulation of sporulation resulting in formation of a cellular spore [GO:0042174], GO:0043940, GO:0043943, positive regulation of sporulation resulting in formation of a cellular spore [GO:0045881] Relationships: is a type of GO:0043937; regulates sporulation resulting in formation of a cellular spore [GO:0030435] Definition: Any process that modulates the frequency, rate or extent of spore formation.